{
  "gene_symbol": "ZNF613",
  "term_id": "GO:0000978",
  "gene": "UniProtKB:Q6PF04",
  "gene_name": "Zinc finger protein 613",
  "term_label": "RNA polymerase II cis-regulatory region sequence-specific DNA binding"
}